{
  "gene_name": "Transcription factor GATA-4",
  "gene": "UniProtKB:P43694",
  "term_id": "GO:0045165",
  "gene_symbol": "GATA4",
  "term_label": "cell fate commitment"
}